endoplasmic reticulum to cytosol auxin transport [GO:0080162] (biological process) Relationships: is a type of transmembrane transport [GO:0055085]; is a type of auxin transport [GO:0060918] Also known as: intracellular auxin transport References: PMID:19506555 Definition: The directed movement of auxins from endoplasmic reticulum to cytosol.